piRNA transcription [GO:0140541] (BP) Regulation: regulated by GO:0140542; positively regulated by positive regulation of piRNA transcription [GO:0140543] Definition: The cellular synthesis of Piwi-interacting RNA piRNAs, a class of 24- to 30-nucleotide RNA derived from repeat or complex DNA sequence elements and processed by a Dicer-independent mechanism. Also known as: PIWI-interacting RNA transcription, Piwi-associated RNA transcription Relationships: is a type of GO:0006351 References: PMID:28847004